{
  "gene_symbol": "ADISSP",
  "gene_name": "Adipose-secreted signaling protein",
  "gene": "UniProtKB:Q9GZN8",
  "term_id": "UNKNOWN:0001",
  "term_label": "Unknown molecular function"
}